specification of carpel identity [GO:0010094] (biological process) Definition: The process in which a floral organ primordium acquires the carpel identity. Identity is considered to be the aggregate of characteristics by which a structure is recognized. Relationships: is a type of specification of floral organ identity [GO:0010093]; is part of carpel formation [GO:0048462] Sources: GOC:tair_curators